pantothenoylcysteine decarboxylase activity [GO:0050167] (molecular function) Definition: Catalysis of the reaction: N-[(R)-pantothenoyl]-L-cysteine + H+ = (R)-pantetheine + CO2. Sources: EC:4.1.1.30, RHEA:15077 Also known as: N-((R)-pantothenoyl)-L-cysteine carboxy-lyase activity, N-[(R)-pantothenoyl]-L-cysteine carboxy-lyase (pantetheine-forming), N-[(R)-pantothenoyl]-L-cysteine carboxy-lyase activity, pantothenylcysteine decarboxylase activity Relationships: is a type of carboxy-lyase activity [GO:0016831]